{
  "gene_name": "Alpha-tocopherol transfer protein",
  "gene": "UniProtKB:P49638",
  "gene_symbol": "TTPA",
  "term_id": "GO:0042360",
  "term_label": "vitamin E metabolic process"
}